negative regulation of reactive oxygen species biosynthetic process [GO:1903427] (biological process) Relationships: is a type of GO:0009890; is a type of regulation of reactive oxygen species biosynthetic process [GO:1903426]; is a type of negative regulation of reactive oxygen species metabolic process [GO:2000378]; negatively regulates reactive oxygen species biosynthetic process [GO:1903409] Also known as: down regulation of reactive oxygen species anabolism, down regulation of reactive oxygen species biosynthesis, down regulation of reactive oxygen species biosynthetic process, down regulation of reactive oxygen species formation, down regulation of reactive oxygen species synthesis, down-regulation of reactive oxygen species anabolism, down-regulation of reactive oxygen species biosynthesis, down-regulation of reactive oxygen species biosynthetic process, down-regulation of reactive oxygen species formation, down-regulation of reactive oxygen species synthesis, downregulation of reactive oxygen species anabolism, downregulation of reactive oxygen species biosynthesis, downregulation of reactive oxygen species biosynthetic process, downregulation of reactive oxygen species formation, downregulation of reactive oxygen species synthesis, negative regulation of reactive oxygen species anabolism, negative regulation of reactive oxygen species biosynthesis, negative regulation of reactive oxygen species formation, negative regulation of reactive oxygen species synthesis, prevention of ROS generation, inhibition of reactive oxygen species anabolism, inhibition of reactive oxygen species biosynthesis, inhibition of reactive oxygen species biosynthetic process, inhibition of reactive oxygen species formation, inhibition of reactive oxygen species synthesis, down regulation of ROS formation, down regulation of ROS generation, down regulation of reactive oxygen species generation, down-regulation of ROS formation, down-regulation of ROS generation, down-regulation of reactive oxygen species generation, downregulation of ROS formation, downregulation of ROS generation, downregulation of reactive oxygen species generation, inhibition of ROS formation, inhibition of ROS generation, inhibition of reactive oxygen species generation, negative regulation of ROS formation, negative regulation of ROS generation, negative regulation of reactive oxygen species generation References: PMID:24252804 Sources: GOC:PARL, GOC:TermGenie, GOC:bf, GO_REF:0000058 Definition: Any process that stops, prevents or reduces the frequency, rate or extent of reactive oxygen species biosynthetic process. Subtypes: GO:0010730